{
  "gene": "UniProtKB:Q5TB80",
  "gene_name": "Centrosomal protein of 162 kDa",
  "term_label": "cilium assembly",
  "term_id": "GO:0060271",
  "gene_symbol": "CEP162"
}